{
  "term_label": "cilium movement involved in cell motility",
  "gene_name": "Tektin-2",
  "term_id": "GO:0060294",
  "gene_symbol": "TEKT2",
  "gene": "UniProtKB:Q9UIF3"
}